regulation of mesenchymal stem cell proliferation involved in nephron morphogenesis [GO:0072042] (biological process) Relationships: is a type of GO:1902460; regulates GO:0072090 Definition: Any process that modulates the frequency, rate or extent of mesenchymal stem cell proliferation and contributes to the shaping of a nephron. Sources: GOC:mtg_kidney_jan10